regulation of T-helper 1 cell differentiation [GO:0045625] (biological process) Also known as: regulation of T-helper 1 cell development Definition: Any process that modulates the frequency, rate or extent of T-helper 1 cell differentiation. Sources: GOC:go_curators Note: Note that immunologists typically use the word 'development' to refer to cells of B or T cell lineages undergoing the process that GO describes as 'cell differentiation'. Subtypes: GO:0045626, GO:0045627 Relationships: is a type of regulation of T-helper 1 type immune response [GO:0002825]; is_a GO:0045622; regulates GO:0045063